{
  "term_label": "phospholipid metabolic process",
  "gene": "UniProtKB:Q7Z2D5",
  "term_id": "GO:0006644",
  "gene_name": "Phospholipid phosphatase-related protein type 4",
  "gene_symbol": "PLPPR4"
}